ABIN2-NFKB1-MAP3K8 complex [GO:0034977] (cellular component) References: PMID:15169888 Also known as: ABIN2-NFKB1-TPL-1 complex Relationships: is a type of intracellular protein-containing complex [GO:0140535]; is a type of GO:1902554 Definition: A protein complex that contains the precursor form of NF-kappaB (p105), the NF-kappaB inhibitor ABIN-2, and the kinase TPL-2 (MAP3K8); the complex stabilizes TPL-2 and is involved in signaling in lipopolysaccharide (LPS)-stimulated macrophages.